{
  "gene_symbol": "IGFL1",
  "term_label": "extracellular space",
  "gene_name": "Insulin growth factor-like family member 1",
  "gene": "UniProtKB:Q6UW32",
  "term_id": "GO:0005615"
}